{
  "gene": "UniProtKB:Q9ULJ8",
  "gene_symbol": "PPP1R9A",
  "gene_name": "Neurabin-1",
  "term_id": "GO:0015629",
  "term_label": "actin cytoskeleton"
}